{
  "term_id": "GO:0061001",
  "gene_name": "Rho GTPase-activating protein 44",
  "gene": "UniProtKB:Q17R89",
  "gene_symbol": "ARHGAP44",
  "term_label": "regulation of dendritic spine morphogenesis"
}